{
  "term_id": "GO:0007254",
  "term_label": "JNK cascade",
  "gene_symbol": "MAPK8",
  "gene": "UniProtKB:P45983",
  "gene_name": "Mitogen-activated protein kinase 8"
}